monoterpenoid biosynthetic process [GO:0016099] (BP) Also known as: monoterpenoid anabolism, monoterpenoid biosynthesis, monoterpenoid formation, monoterpenoid synthesis Definition: The chemical reactions and pathways resulting in the formation of monoterpenoid compounds, terpenoids having a C10 skeleton. Subtypes: menthol biosynthetic process [GO:0031525], GO:0046211, (-)-secologanin biosynthetic process [GO:1900994], geraniol biosynthetic process [GO:1903448] Relationships: is a type of monoterpenoid metabolic process [GO:0016098]; is a type of terpenoid biosynthetic process [GO:0016114] Sources: GOC:go_curators